miltiradiene synthase activity [GO:0062205] (molecular function) Also known as: multiradiene synthase activity Definition: Catalysis of the reaction: (+)-copalyl diphosphate = diphosphate + miltiradiene. Relationships: is a type of carbon-oxygen lyase activity, acting on phosphates [GO:0016838] References: PMID:24990389 Sources: RHEA:33983